development of primary sexual characteristics [GO:0045137] (biological process) Relationships: is a type of developmental process involved in reproduction [GO:0003006]; is part of multicellular organism development [GO:0007275]; is part of sex differentiation [GO:0007548] Sources: GOC:ai Definition: The process whose specific outcome is the progression of the primary sexual characteristics over time, from their formation to the mature structures. The primary sexual characteristics are the testes in males and the ovaries in females and they develop in response to sex hormone secretion. Subtypes: development of primary female sexual characteristics [GO:0046545], development of primary male sexual characteristics [GO:0046546]